{
  "gene": "UniProtKB:Q9Y5L3",
  "gene_symbol": "ENTPD2",
  "term_id": "GO:0009134",
  "gene_name": "Ectonucleoside triphosphate diphosphohydrolase 2",
  "term_label": "nucleoside diphosphate catabolic process"
}